methylcrotonoyl-CoA carboxylase activity [GO:0004485] (molecular function) Definition: Catalysis of the reaction: 3-methylbut-2-enoyl-CoA + ATP + bicarbonate = trans-3-methylglutaconyl-CoA + ADP + 2 H+ + phosphate. Relationships: is a type of CoA carboxylase activity [GO:0016421] Also known as: MCCC activity, 3-methylcrotonoyl-CoA:carbon-dioxide ligase (ADP-forming), beta-methylcrotonyl CoA carboxylase activity, beta-methylcrotonyl coenzyme A carboxylase activity, beta-methylcrotonyl-CoA carboxylase activity, methylcrotonyl coenzyme A carboxylase activity, methylcrotonyl-CoA carboxylase activity Sources: EC:6.4.1.4, RHEA:13589